neurotrophin production [GO:0032898] (biological process) Relationships: is a type of multicellular organismal process [GO:0032501] Sources: GOC:ecd, GOC:mah, GOC:mtg_MIT_16mar07 Regulation: RO_0002211 by GO:0032899; negatively regulated by negative regulation of neurotrophin production [GO:0032900]; positively regulated by positive regulation of neurotrophin production [GO:0032901] Definition: The appearance of a neurotrophin due to biosynthesis or secretion by cells in a neuron's target field, resulting in an increase in its intracellular or extracellular levels. A neurotrophin is any of a family of growth factors that prevent apoptosis in neurons and promote nerve growth. Subtypes: nerve growth factor production [GO:0032902]